parietal peritoneum development [GO:1904819] (biological process) References: PMID:15840053 Sources: GOC:TermGenie, GOC:dph, GO_REF:0000094 Also known as: peritoneal cavity lining development Relationships: is a type of anatomical structure development [GO:0048856]; is part of peritoneum development [GO:1904820] Definition: The process whose specific outcome is the progression of a parietal peritoneum over time, from its formation to the mature structure.